{
  "gene_symbol": "AICDA",
  "term_label": "cytidine deaminase activity",
  "gene": "UniProtKB:Q9GZX7",
  "gene_name": "Single-stranded DNA cytosine deaminase",
  "term_id": "GO:0004126"
}